{
  "term_label": "peptide antigen assembly with MHC class II protein complex",
  "term_id": "GO:0002503",
  "gene": "UniProtKB:P79483",
  "gene_name": "HLA class II histocompatibility antigen, DR beta 3 chain",
  "gene_symbol": "HLA-DRB3"
}